{
  "gene_symbol": "CHD6",
  "term_id": "GO:0042393",
  "gene_name": "Chromodomain-helicase-DNA-binding protein 6",
  "gene": "UniProtKB:Q8TD26",
  "term_label": "histone binding"
}